toll-like receptor 1 signaling pathway [GO:0034130] (biological process) Regulation: regulated by regulation of toll-like receptor 1 signaling pathway [GO:0034131]; negatively regulated by negative regulation of toll-like receptor 1 signaling pathway [GO:0034132]; positively regulated by positive regulation of toll-like receptor 1 signaling pathway [GO:0034133] Definition: The series of molecular signals initiated by a ligand binding to toll-like receptor 1. Relationships: is a type of cell surface pattern recognition receptor signaling pathway [GO:0002752] References: PMID:16551253, PMID:17328678 Sources: GOC:add Also known as: TLR1 signaling pathway, toll-like receptor 1 signalling pathway